gentamycin metabolic process [GO:1901128] (biological process) Definition: The chemical reactions and pathways involving gentamycin. Sources: GOC:TermGenie, GOC:yaf, UniPathway:UPA00967 Also known as: gentamycin metabolism Relationships: is a type of glycoside metabolic process [GO:0016137]; is_a GO:0019751 Subtypes: gentamycin catabolic process [GO:1901129], gentamycin biosynthetic process [GO:1901130]